{
  "gene_symbol": "A0A6Q8PFC9",
  "term_id": "UNKNOWN:0003",
  "gene": "UniProtKB:A0A6Q8PFC9",
  "term_label": "Unknown cellular component",
  "gene_name": "Uncharacterized protein"
}